{
  "term_label": "Unknown molecular function",
  "gene": "UniProtKB:P04435",
  "term_id": "UNKNOWN:0001",
  "gene_name": "T cell receptor beta variable 7-9",
  "gene_symbol": "TRBV7-9"
}